{
  "gene_symbol": "SUPT6H",
  "term_label": "histone binding",
  "term_id": "GO:0042393",
  "gene_name": "Transcription elongation factor SPT6",
  "gene": "UniProtKB:Q7KZ85"
}